{
  "gene_name": "Neurotrypsin",
  "term_id": "GO:0005886",
  "gene": "UniProtKB:P56730",
  "term_label": "plasma membrane",
  "gene_symbol": "PRSS12"
}